{
  "gene_name": "M-phase inducer phosphatase 3",
  "term_label": "protein tyrosine phosphatase activity",
  "gene_symbol": "CDC25C",
  "gene": "UniProtKB:P30307",
  "term_id": "GO:0004725"
}